{
  "term_label": "proton motive force-driven ATP synthesis",
  "gene_symbol": "ATP5PB",
  "gene_name": "ATP synthase F(0) complex subunit B1, mitochondrial",
  "term_id": "GO:0015986",
  "gene": "UniProtKB:P24539"
}